{
  "gene_symbol": "FAHD1",
  "term_label": "Unknown biological process",
  "term_id": "UNKNOWN:0002",
  "gene": "UniProtKB:Q6P587",
  "gene_name": "Acylpyruvase FAHD1, mitochondrial"
}